calcium-mediated signaling [GO:0019722] (biological process) Sources: GOC:signaling Also known as: calcium ion signaling, calcium signaling, calcium signalling, calcium-mediated signalling Relationships: is a type of GO:0141124 Subtypes: regulation of cardiac muscle contraction by calcium ion signaling [GO:0010882], regulation of skeletal muscle contraction by calcium ion signaling [GO:0014722], GO:0061762, calcineurin-mediated signaling [GO:0097720] Regulation: regulated by regulation of calcium-mediated signaling [GO:0050848]; negatively regulated by negative regulation of calcium-mediated signaling [GO:0050849]; positively regulated by positive regulation of calcium-mediated signaling [GO:0050850] Definition: Any intracellular signal transduction in which the signal is passed on within the cell via calcium ions.